{
  "term_label": "Unknown biological process",
  "gene_symbol": "TRAJ45",
  "term_id": "UNKNOWN:0002",
  "gene_name": "T cell receptor alpha joining 45 (Fragment)",
  "gene": "UniProtKB:A0A075B6X0"
}